negative regulation of calcium-dependent ATPase activity [GO:1903611] (biological process) Relationships: is a type of GO:0032780; negatively regulates GO:0030899 Also known as: down regulation of calcium-dependent ATPase activity, down-regulation of calcium-dependent ATPase activity, downregulation of calcium-dependent ATPase activity, inhibition of calcium-dependent ATPase activity References: PMID:10861851 Sources: GOC:TermGenie, GO_REF:0000059 Definition: Any process that stops, prevents or reduces the frequency, rate or extent of calcium-dependent ATPase activity.